positive regulation of hexadecanal biosynthetic process [GO:1900904] (biological process) Also known as: up regulation of hexadecanal biosynthetic process, up-regulation of hexadecanal biosynthetic process, upregulation of hexadecanal biosynthetic process, activation of hexadecanal anabolism, activation of hexadecanal biosynthesis, activation of hexadecanal biosynthetic process, activation of hexadecanal formation, activation of hexadecanal synthesis, activation of palmitaldehyde biosynthesis, activation of palmitaldehyde biosynthetic process, positive regulation of hexadecanal anabolism, positive regulation of hexadecanal biosynthesis, positive regulation of hexadecanal formation, positive regulation of hexadecanal synthesis, positive regulation of palmitaldehyde biosynthesis, positive regulation of palmitaldehyde biosynthetic process, up regulation of hexadecanal anabolism, up regulation of hexadecanal biosynthesis, up regulation of hexadecanal formation, up regulation of hexadecanal synthesis, up regulation of palmitaldehyde biosynthesis, up regulation of palmitaldehyde biosynthetic process, up-regulation of hexadecanal anabolism, up-regulation of hexadecanal biosynthesis, up-regulation of hexadecanal formation, up-regulation of hexadecanal synthesis, up-regulation of palmitaldehyde biosynthesis, up-regulation of palmitaldehyde biosynthetic process, upregulation of hexadecanal anabolism, upregulation of hexadecanal biosynthesis, upregulation of hexadecanal formation, upregulation of hexadecanal synthesis, upregulation of palmitaldehyde biosynthesis, upregulation of palmitaldehyde biosynthetic process Definition: Any process that activates or increases the frequency, rate or extent of hexadecanal biosynthetic process. Relationships: is a type of positive regulation of biosynthetic process [GO:0009891]; is a type of regulation of hexadecanal biosynthetic process [GO:1900902]; RO_0002213 hexadecanal biosynthetic process [GO:0006634] Sources: GOC:TermGenie, GOC:mengo_curators